{
  "term_label": "COPI-coated vesicle",
  "gene_name": "Transmembrane emp24 domain-containing protein 10",
  "gene": "UniProtKB:P49755",
  "gene_symbol": "TMED10",
  "term_id": "GO:0030137"
}